{
  "term_id": "GO:0007165",
  "gene_name": "Protein NDRG3",
  "term_label": "signal transduction",
  "gene": "UniProtKB:Q9UGV2",
  "gene_symbol": "NDRG3"
}